{
  "term_label": "mitochondrion",
  "gene_symbol": "SDHAF3",
  "gene": "UniProtKB:Q9NRP4",
  "gene_name": "Succinate dehydrogenase assembly factor 3, mitochondrial",
  "term_id": "GO:0005739"
}